{
  "term_label": "Unknown biological process",
  "gene_symbol": "RPS15A",
  "gene_name": "Small ribosomal subunit protein uS8",
  "gene": "UniProtKB:P62244",
  "term_id": "UNKNOWN:0002"
}